{
  "gene_name": "Voltage-dependent N-type calcium channel subunit alpha-1B",
  "gene_symbol": "CACNA1B",
  "term_id": "GO:0043025",
  "term_label": "neuronal cell body",
  "gene": "UniProtKB:Q00975"
}